{
  "gene_name": "Proline_serine-rich coiled-coil protein 1",
  "term_label": "mitotic metaphase chromosome alignment",
  "term_id": "GO:0007080",
  "gene": "UniProtKB:Q6PGN9",
  "gene_symbol": "PSRC1"
}